type 4 somatostatin receptor binding [GO:0031881] (molecular function) Sources: GOC:mah, GOC:nln Relationships: is a type of somatostatin receptor binding [GO:0031877] Also known as: type 4 somatostatin receptor ligand Definition: Binding to a type 4 somatostatin receptor.